carbohydrate export [GO:0033231] (biological process) Relationships: is a type of carbohydrate transport [GO:0008643] Definition: The directed movement of carbohydrates out of a cell or organelle. Sources: GOC:mlg